{
  "gene": "UniProtKB:P22891",
  "gene_symbol": "PROZ",
  "gene_name": "Vitamin K-dependent protein Z",
  "term_id": "GO:0007596",
  "term_label": "blood coagulation"
}